positive regulation of dense core granule transport [GO:1904811] (biological process) Also known as: positive regulation of dense core vesicle transport, up regulation of dense core granule transport, up regulation of dense core vesicle transport, up-regulation of dense core granule transport, up-regulation of dense core vesicle transport, upregulation of dense core granule transport, upregulation of dense core vesicle transport, activation of dense core granule transport, activation of dense core vesicle transport References: PMID:22699897 Sources: GOC:TermGenie, GO_REF:0000058 Subtypes: positive regulation of anterograde dense core granule transport [GO:1901953], positive regulation of retrograde dense core granule transport [GO:1901956] Note: cdk-5 in C.elegans (G5ECH7) in PMID:22699897 (inferred from mutant phenotype). Definition: Any process that activates or increases the frequency, rate or extent of dense core granule transport. Relationships: is a type of positive regulation of intracellular transport [GO:0032388]; is a type of GO:1904809; positively regulates dense core granule transport [GO:1901950]